{
  "gene_symbol": "H2BC21",
  "gene_name": "Histone H2B type 2-E",
  "gene": "UniProtKB:Q16778",
  "term_id": "GO:0019731",
  "term_label": "antibacterial humoral response"
}